{
  "gene": "UniProtKB:Q19AV6",
  "gene_name": "Zinc finger SWIM domain-containing protein 7",
  "gene_symbol": "ZSWIM7",
  "term_label": "Shu complex",
  "term_id": "GO:0097196"
}